{
  "gene": "UniProtKB:Q16799",
  "gene_symbol": "RTN1",
  "term_label": "neuron projection",
  "gene_name": "Reticulon-1",
  "term_id": "GO:0043005"
}